NMDA glutamate receptor activity [GO:0004972] (molecular function) Relationships: is a type of glutamate-gated receptor activity [GO:0004970]; is a type of GO:0005244 Regulation: negatively regulated by GO:1904782; regulated by GO:2000310 Definition: A cation channel that opens in response to binding by extracellular glutmate, but only if glycine or D-serine is also bound and the membrane is depolarized. Voltage gating is indirect, due to ejection of bound magnesium from the pore at permissive voltages. References: PMID:10049997, PMID:7790891 Sources: GOC:mah Note: The name of this receptor comes from its selective activation by N-methyl-D-aspartate (NMDA). Note that this term represents an activity and not a gene product. Also known as: N-methyl-D-aspartate selective glutamate receptor activity, NMDA receptor